lipoate biosynthetic process [GO:0009107] (biological process) Definition: The chemical reactions and pathways resulting in the formation of lipoate, 1,2-dithiolane-3-pentanoate, the anion derived from lipoic acid. Sources: GOC:ai, ISBN:0198506732 Also known as: lipoate anabolism, lipoate biosynthesis, lipoate formation, lipoate synthesis, lipoic acid anabolism, lipoic acid biosynthesis, lipoic acid biosynthetic process, lipoic acid formation, lipoic acid synthesis Relationships: is a type of fatty acid biosynthetic process [GO:0006633]; is a type of lipoate metabolic process [GO:0009106]; is_a sulfur compound biosynthetic process [GO:0044272]